intracellular nickel ion homeostasis [GO:0035785] (biological process) Also known as: cellular nickel homeostasis, cellular nickel ion homeostasis Relationships: is a type of GO:0030003; is a type of inorganic ion homeostasis [GO:0098771] Definition: A homeostatic process involved in the maintenance of a steady state level of nickel ions within a cell. Sources: GOC:kmv